{
  "gene": "UniProtKB:A0A0K0K1A3",
  "term_label": "cell surface receptor signaling pathway",
  "gene_symbol": "TRBV10-1",
  "gene_name": "T cell receptor beta variable 10-1",
  "term_id": "GO:0007166"
}